{
  "gene": "UniProtKB:P78325",
  "gene_symbol": "ADAM8",
  "gene_name": "Disintegrin and metalloproteinase domain-containing protein 8",
  "term_label": "metalloendopeptidase activity",
  "term_id": "GO:0004222"
}